regulation of retrograde transport, endosome to Golgi [GO:1905279] (biological process) Relationships: is a type of regulation of intracellular transport [GO:0032386]; is a type of GO:0060627; regulates retrograde transport, endosome to Golgi [GO:0042147] Also known as: regulation of retrograde (endosome to Golgi) transport References: PMID:23395371 Sources: GOC:PARL, GOC:TermGenie, GOC:bf, GO_REF:0000058 Definition: Any process that modulates the frequency, rate or extent of retrograde transport, endosome to Golgi. Subtypes: negative regulation of retrograde transport, endosome to Golgi [GO:1905280], positive regulation of retrograde transport, endosome to Golgi [GO:1905281]